{
  "term_id": "GO:0043025",
  "gene_name": "Hemicentin-2",
  "term_label": "neuronal cell body",
  "gene_symbol": "HMCN2",
  "gene": "UniProtKB:Q8NDA2"
}